{
  "gene": "UniProtKB:Q9GZK3",
  "gene_name": "Olfactory receptor 2B2",
  "gene_symbol": "OR2B2",
  "term_label": "detection of chemical stimulus involved in sensory perception of smell",
  "term_id": "GO:0050911"
}